flavone 7-O-beta-glucosyltransferase activity [GO:0047891] (molecular function) Definition: Catalysis of the reaction: UDP-glucose + 5,7,3',4'-tetrahydroxyflavone = UDP + 7-O-beta-D-glucosyl-5,7,3',4'-tetrahydroxyflavone. Sources: EC:2.4.1.81, MetaCyc:FLAVONE-7-O-BETA-GLUCOSYLTRANSFERASE-RXN Also known as: flavone 7-O-b-glucosyltransferase activity, UDP-glucose-apigenin beta-glucosyltransferase activity, UDP-glucose-luteolin beta-D-glucosyltransferase activity, UDP-glucose:5,7,3',4'-tetrahydroxyflavone 7-O-beta-D-glucosyltransferase activity, UDPglucose-apigenin beta-glucosyltransferase activity, UDPglucose-luteolin beta-D-glucosyltransferase activity, UDPglucose:5,7,3',4'-tetrahydroxyflavone 7-O-beta-D-glucosyltransferase activity, uridine diphosphoglucose-apigenin 7-O-glucosyltransferase activity, uridine diphosphoglucose-luteolin glucosyltransferase activity Relationships: is a type of UDP-glucosyltransferase activity [GO:0035251]